juvenile-hormone esterase activity [GO:0004453] (molecular function) Relationships: is a type of carboxylic ester hydrolase activity [GO:0052689] References: PMID:11267890 Sources: RHEA:16393 Also known as: JH esterase activity, JH-esterase activity, juvenile hormone analog esterase activity, juvenile hormone carboxyesterase activity, methyl-(2E,6E)-(10R,11S)-10,11-epoxy-3,7,11-trimethyltrideca-2,6-dienoate acylhydrolase activity Definition: Catalysis of the reaction: methyl (2E,6E)-(10R,11S)-10,11-epoxy-3,7,11-trimethyltrideca-2,6-dienoate + H2O = (2E,6E)-(10R,11S)-10,11-epoxy-3,7,11-trimethyltrideca-2,6-dienoate + methanol. A carboxylesterase that hydrolyzes the ester linkage of juvenile hormone.